{
  "term_label": "Unknown cellular component",
  "term_id": "UNKNOWN:0003",
  "gene_symbol": "ZNF718",
  "gene_name": "Zinc finger protein 718",
  "gene": "UniProtKB:Q3SXZ3"
}